AMP deaminase activity [GO:0003876] (molecular function) Definition: Catalysis of the reaction: AMP + H2O = IMP + NH3. Relationships: is a type of adenosine-phosphate deaminase activity [GO:0047623] Also known as: adenylate deaminase reaction, myoadenylate deaminase activity, 5-AMP deaminase activity, 5-adenylate deaminase activity, 5-adenylic acid deaminase activity, AMP aminase activity, AMP aminohydrolase activity, adenosine 5-monophosphate deaminase activity, adenosine 5-phosphate aminohydrolase activity, adenosine monophosphate deaminase activity, adenyl deaminase activity, adenylate aminohydrolase activity, adenylate deaminase activity, adenylate desaminase activity, adenylic acid deaminase activity, adenylic deaminase activity Sources: EC:3.5.4.6